{
  "gene": "UniProtKB:Q6ZUJ8",
  "gene_symbol": "PIK3AP1",
  "term_id": "UNKNOWN:0002",
  "term_label": "Unknown biological process",
  "gene_name": "Phosphoinositide 3-kinase adapter protein 1"
}